{
  "gene_symbol": "A0A6Q8PHS2",
  "gene_name": "Uncharacterized protein",
  "term_label": "Unknown cellular component",
  "term_id": "UNKNOWN:0003",
  "gene": "UniProtKB:A0A6Q8PHS2"
}